ceramide translocation [GO:0099040] (biological process) Definition: The movement of a ceramide molecule from one leaflet of a membrane bilayer to the opposite leaflet. Sources: GOC:BHF, GOC:rl Relationships: is a type of ceramide transport [GO:0035627]; is a type of sphingolipid translocation [GO:0099039]